negative regulation of intermediate mesodermal cell fate determination [GO:0048396] (biological process) Also known as: down regulation of intermediate mesodermal cell fate determination, down-regulation of intermediate mesodermal cell fate determination, downregulation of intermediate mesodermal cell fate determination, inhibition of intermediate mesodermal cell fate determination Relationships: is_a negative regulation of mesodermal cell fate determination [GO:0048335]; is a type of GO:0048395; negatively regulates intermediate mesodermal cell fate determination [GO:0048394] Definition: Any process that stops, prevents, or reduces the frequency, rate or extent of intermediate mesoderm cell fate determination. Sources: GOC:dgh